{
  "gene": "UniProtKB:Q9Y2K1",
  "gene_symbol": "ZBTB1",
  "term_label": "negative regulation of transcription by RNA polymerase II",
  "term_id": "GO:0000122",
  "gene_name": "Zinc finger and BTB domain-containing protein 1"
}